{
  "term_id": "GO:0099530",
  "gene_symbol": "GRM1",
  "term_label": "G protein-coupled receptor activity involved in regulation of postsynaptic membrane potential",
  "gene_name": "Metabotropic glutamate receptor 1",
  "gene": "UniProtKB:Q13255"
}